{
  "gene_symbol": "PLAAT4",
  "term_label": "phospholipase A1 activity",
  "gene": "UniProtKB:Q9UL19",
  "term_id": "GO:0008970",
  "gene_name": "Phospholipase A and acyltransferase 4"
}